{
  "term_id": "GO:0005251",
  "term_label": "delayed rectifier potassium channel activity",
  "gene_symbol": "KCNA7",
  "gene_name": "Potassium voltage-gated channel subfamily A member 7",
  "gene": "UniProtKB:Q96RP8"
}